{
  "gene_symbol": "PLPP5",
  "gene": "UniProtKB:Q8NEB5",
  "term_label": "phospholipid metabolic process",
  "term_id": "GO:0006644",
  "gene_name": "Phospholipid phosphatase 5"
}